6-carboxyhexanoate-CoA ligase activity [GO:0042410] (MF) Sources: EC:6.2.1.14, RHEA:14781 Definition: Catalysis of the reaction: ATP + CoA + pimelate = AMP + diphosphate + H+ + pimelyl-CoA. Relationships: is a type of CoA-ligase activity [GO:0016405]; is a type of acid-thiol ligase activity [GO:0016878] Also known as: 6-carboxyhexanoate:CoA ligase (AMP-forming), 6-carboxyhexanoyl-CoA synthetase activity, pimeloyl-CoA synthetase activity, pimelyl-CoA synthetase activity